{
  "gene_name": "G patch domain-containing protein 4",
  "term_id": "UNKNOWN:0002",
  "gene_symbol": "GPATCH4",
  "gene": "UniProtKB:Q5T3I0",
  "term_label": "Unknown biological process"
}